viral DNA genome packaging via site-specific sequence recognition [GO:0098035] (biological process) Definition: The encapsulation of the viral DNA genome within the capsid, which proceeds via cleavage of the viral DNA at specific sites by a viral terminase. Subtypes: viral DNA genome packaging, 3' extended cos packaging [GO:0098036], viral DNA genome packaging, 5' extended cos packaging [GO:0098037] Sources: GOC:bm Regulation: regulated by regulation of viral DNA genome packaging via site-specific sequence recognition [GO:1905137]; positively regulated by positive regulation of viral DNA genome packaging via site-specific sequence recognition [GO:1905138] Relationships: is a type of viral DNA genome packaging [GO:0019073]